positive regulation of lung goblet cell differentiation [GO:1901251] (biological process) Also known as: positive regulation of pulmonary goblet cell differentiation, up regulation of lung goblet cell differentiation, up regulation of pulmonary goblet cell differentiation, up-regulation of lung goblet cell differentiation, up-regulation of pulmonary goblet cell differentiation, upregulation of lung goblet cell differentiation, upregulation of pulmonary goblet cell differentiation, activation of lung goblet cell differentiation, activation of pulmonary goblet cell differentiation Relationships: is a type of positive regulation of epithelial cell differentiation [GO:0030858]; is_a positive regulation of multicellular organismal process [GO:0051240]; is a type of regulation of lung goblet cell differentiation [GO:1901249]; positively regulates lung goblet cell differentiation [GO:0060480] Sources: GOC:BHF, GOC:TermGenie Definition: Any process that activates or increases the frequency, rate or extent of lung goblet cell differentiation.